{
  "term_id": "GO:0035556",
  "gene": "UniProtKB:Q9Y376",
  "term_label": "intracellular signal transduction",
  "gene_symbol": "CAB39",
  "gene_name": "Calcium-binding protein 39"
}